{
  "gene_name": "Tigger transposable element-derived protein 7",
  "gene_symbol": "TIGD7",
  "gene": "UniProtKB:Q6NT04",
  "term_label": "nucleus",
  "term_id": "GO:0005634"
}